sucrose 6F-alpha-galactotransferase activity [GO:0047235] (molecular function) Definition: Catalysis of the reaction: sucrose + UDP-galactose = 6F-alpha-D-galactosylsucrose + UDP. Sources: EC:2.4.1.167, MetaCyc:2.4.1.167-RXN Also known as: sucrose 6(F)-alpha-galactosyltransferase activity, UDP-galactose:sucrose 6F-alpha-D-galactosyltransferase activity, UDPgalactose:sucrose 6F-alpha-D-galactosyltransferase activity, UDPgalactose:sucrose 6fru-alpha-galactosyltransferase activity, sucrose 6F-alpha-galactosyltransferase activity, uridine diphosphogalactose-sucrose 6F-alpha-galactosyltransferase activity Relationships: is a type of UDP-galactosyltransferase activity [GO:0035250]